T cell costimulation [GO:0031295] (biological process) Definition: The process of providing, via surface-bound receptor-ligand pairs, a second, antigen-independent, signal in addition to that provided by the T cell receptor to augment T cell activation. Sources: ISBN:0781735149 Also known as: T cell co-stimulation, T lymphocyte costimulation, T-cell co-stimulation, T-cell costimulation, T-lymphocyte costimulation Relationships: is a type of GO:0031294; is a type of GO:0050870 Subtypes: GO:0035783 Regulation: regulated by regulation of T cell costimulation [GO:2000523]; negatively regulated by negative regulation of T cell costimulation [GO:2000524]; positively regulated by positive regulation of T cell costimulation [GO:2000525]